{
  "gene_name": "Cytidine deaminase",
  "term_label": "cytidine deaminase activity",
  "gene": "UniProtKB:P32320",
  "term_id": "GO:0004126",
  "gene_symbol": "CDA"
}